C-C chemokine binding [GO:0019957] (molecular function) Relationships: is a type of chemokine binding [GO:0019956] Sources: GOC:ai Definition: Binding to a C-C chemokine; C-C chemokines do not have an amino acid between the first two cysteines of the characteristic four-cysteine motif. Subtypes: chemokine (C-C motif) ligand 2 binding [GO:0035715], chemokine (C-C motif) ligand 12 binding [GO:0035716], GO:0035717, chemokine (C-C motif) ligand 19 binding [GO:0035757], chemokine (C-C motif) ligand 21 binding [GO:0035758], chemokine (C-C motif) ligand 5 binding [GO:0071791]